{
  "term_label": "Golgi stack",
  "gene_symbol": "NSF",
  "term_id": "GO:0005795",
  "gene_name": "Vesicle-fusing ATPase",
  "gene": "UniProtKB:P46459"
}